{
  "term_label": "Unknown molecular function",
  "gene_name": "Putative uncharacterized protein FLJ40288",
  "gene_symbol": "A4D1N5",
  "term_id": "UNKNOWN:0001",
  "gene": "UniProtKB:A4D1N5"
}